detection of chemical stimulus involved in sensory perception of pain [GO:0050968] (biological process) Definition: The series of events involved in the perception of pain in which a chemical stimulus is received and converted into a molecular signal. Also known as: perception of pain, detection of chemical stimulus, perception of pain, sensory detection of chemical stimulus, perception of pain, sensory transduction of chemical stimulus, sensory detection of chemical stimulus during perception of pain, sensory transduction of chemical stimulus during perception of pain, chemical nociception Relationships: is a type of detection of chemical stimulus involved in sensory perception [GO:0050907]; is a type of detection of stimulus involved in sensory perception of pain [GO:0062149] Sources: GOC:ai